secretin receptor activity [GO:0015055] (molecular function) Sources: GOC:mah Definition: Combining with secretin to initiate a change in cell activity. Relationships: is a type of G protein-coupled receptor activity [GO:0004930]